{
  "gene": "UniProtKB:P28370",
  "term_id": "GO:0140750",
  "gene_name": "Probable global transcription activator SNF2L1",
  "term_label": "nucleosome array spacer activity",
  "gene_symbol": "SMARCA1"
}